dimethylallyl diphosphate biosynthetic process [GO:0050992] (biological process) Also known as: DPP biosynthesis, DPP biosynthetic process, dimethylallyl diphosphate anabolism, dimethylallyl diphosphate biosynthesis, dimethylallyl diphosphate formation, dimethylallyl diphosphate synthesis, dimethylallyl pyrophosphate biosynthesis, dimethylallyl pyrophosphate biosynthetic process Relationships: is a type of phospholipid biosynthetic process [GO:0008654]; is a type of GO:0050993 Definition: The chemical reactions and pathways resulting in the formation of dimethylallyl diphosphate. Sources: GOC:ai